{
  "term_label": "Unknown biological process",
  "gene": "UniProtKB:Q4QY38",
  "gene_symbol": "DEFB134",
  "term_id": "UNKNOWN:0002",
  "gene_name": "Beta-defensin 134"
}